{
  "term_label": "membrane",
  "gene_name": "Ras-related protein Rab-10",
  "term_id": "GO:0016020",
  "gene": "UniProtKB:P61026",
  "gene_symbol": "RAB10"
}